{
  "gene_symbol": "TRA2A",
  "gene_name": "Transformer-2 protein homolog alpha",
  "gene": "UniProtKB:Q13595",
  "term_id": "GO:0003729",
  "term_label": "mRNA binding"
}